{
  "gene": "UniProtKB:O14653",
  "gene_name": "Golgi SNAP receptor complex member 2",
  "gene_symbol": "GOSR2",
  "term_id": "GO:0005794",
  "term_label": "Golgi apparatus"
}